{
  "gene": "UniProtKB:O60437",
  "term_id": "GO:0005737",
  "gene_symbol": "PPL",
  "term_label": "cytoplasm",
  "gene_name": "Periplakin"
}